ABC-type molybdate transporter activity [GO:0015412] (molecular function) Definition: Enables the transfer of a solute or solutes from one side of a membrane to the other according to the reaction: ATP + H2O + molybdate(out) = ADP + phosphate + molybdate(in). Relationships: is a type of GO:0015098; is_a ABC-type transporter activity [GO:0140359] Also known as: molybdate porter activity, molybdate ABC transporter, ATPase-coupled molybdate transmembrane transporter activity, molybdate transmembrane-transporting ATPase activity, molybdate transporting ATPase activity, molybdate-transporting ATPase activity Sources: RHEA:22020